{
  "term_id": "UNKNOWN:0001",
  "gene_symbol": "ECSCR",
  "term_label": "Unknown molecular function",
  "gene_name": "Endothelial cell-specific chemotaxis regulator",
  "gene": "UniProtKB:Q19T08"
}